{
  "gene_symbol": "UTP6",
  "term_id": "GO:0030515",
  "gene_name": "U3 small nucleolar RNA-associated protein 6 homolog",
  "term_label": "snoRNA binding",
  "gene": "UniProtKB:Q9NYH9"
}